{
  "gene": "UniProtKB:Q7Z3K3",
  "term_label": "regulation of DNA-templated transcription",
  "gene_name": "Pogo transposable element with ZNF domain",
  "gene_symbol": "POGZ",
  "term_id": "GO:0006355"
}